{
  "gene": "UniProtKB:Q8N3Z3",
  "term_id": "GO:0005739",
  "gene_name": "GTP-binding protein 8",
  "term_label": "mitochondrion",
  "gene_symbol": "GTPBP8"
}